{
  "gene_name": "Sphingosine kinase 2",
  "term_label": "sphinganine-1-phosphate biosynthetic process",
  "term_id": "GO:0006669",
  "gene_symbol": "SPHK2",
  "gene": "UniProtKB:Q9NRA0"
}